basket cell precursor proliferation [GO:0021928] (biological process) References: PMID:15157725 Sources: GOC:cls, GOC:dgh, GOC:dph, GOC:jid, GO_REF:0000021 Definition: The multiplication or reproduction of neuroblasts that will give rise to basket cells. A cerebellar basket cell is an inhibitory GABAergic interneuron found in the cerebellar cortex. Relationships: is a type of cell proliferation in hindbrain ventricular zone [GO:0021923]